{
  "term_id": "GO:0004711",
  "term_label": "ribosomal protein S6 kinase activity",
  "gene_symbol": "RPS6KA1",
  "gene": "UniProtKB:Q15418",
  "gene_name": "Ribosomal protein S6 kinase alpha-1"
}